polyprenal reductase activity [GO:0160198] (molecular function) Definition: Catalysis of the reaction: ditrans,polycis-polyprenal+ H+ + NADPH = ditrans,polycis-dolichal+ NADP. References: PMID:38821050 Sources: RHEA:80727 Relationships: is a type of oxidoreductase activity, acting on the CH-CH group of donors, NAD or NADP as acceptor [GO:0016628]